{
  "gene_symbol": "SSBP1",
  "term_id": "GO:0042645",
  "gene": "UniProtKB:Q04837",
  "term_label": "mitochondrial nucleoid",
  "gene_name": "Single-stranded DNA-binding protein, mitochondrial"
}